{
  "gene": "UniProtKB:Q15825",
  "gene_name": "Neuronal acetylcholine receptor subunit alpha-6",
  "term_label": "acetylcholine receptor activity",
  "term_id": "GO:0015464",
  "gene_symbol": "CHRNA6"
}